host response to induction by symbiont of tumor, nodule or growth in host [GO:0080034] (biological process) Relationships: is_a response to symbiont [GO:0009608] References: PMID:18836040 Definition: Any process that results in a change in the state or activity of a host cell or organism (in terms of movement, secretion, enzyme production, gene expression, etc.) as a result of the formation of an abnormal mass of cells in the host organism, induced by a symbiont. The host is defined as the larger of the organisms involved in a symbiotic interaction.